negative regulation of axon extension involved in axon guidance [GO:0048843] (biological process) Definition: Any process that stops, prevents, or reduces the frequency, rate or extent of axon extension involved in axon guidance. Sources: GOC:devbiol Also known as: down regulation of axon extension involved in axon guidance, down-regulation of axon extension involved in axon guidance, downregulation of axon extension involved in axon guidance, inhibition of axon extension involved in axon guidance Relationships: is a type of negative regulation of axon extension [GO:0030517]; is a type of regulation of axon extension involved in axon guidance [GO:0048841]; is_a negative regulation of chemotaxis [GO:0050922]; negatively regulates axon extension involved in axon guidance [GO:0048846]